cellular response to thiabendazole [GO:0072713] (biological process) Definition: Any process that results in a change in state or activity of a cell (in terms of movement, secretion, enzyme production, gene expression, etc.) as a result of a thiabendazole stimulus. Relationships: is a type of GO:0072712; is a type of cellular response to nitrogen compound [GO:1901699] Sources: GOC:mah Also known as: cellular response to TBZ